ionotropic salty taste receptor activity [GO:0033039] (molecular function) Definition: Enables the transmembrane transfer of an ion by a channel that opens when a soluble salty compound has been bound by the channel complex or one of its constituent parts. References: PMID:36332657 Sources: GOC:mah Relationships: is a type of ionotropic taste receptor activity [GO:0170021]